{
  "gene": "UniProtKB:Q15349",
  "term_id": "GO:0004711",
  "gene_symbol": "RPS6KA2",
  "gene_name": "Ribosomal protein S6 kinase alpha-2",
  "term_label": "ribosomal protein S6 kinase activity"
}